{
  "gene": "UniProtKB:Q04864",
  "term_id": "GO:0000978",
  "term_label": "RNA polymerase II cis-regulatory region sequence-specific DNA binding",
  "gene_name": "Proto-oncogene c-Rel",
  "gene_symbol": "REL"
}